calcium ion binding involved in regulation of postsynaptic cytosolic calcium ion concentration [GO:0099567] (molecular function) Also known as: calcium ion binding involved in regulation of postsynaptic cytosolic calcium levels, postsynaptic calcium ion buffering, regulation of postsynaptic cytosolic calcium ion concentration by calcium ion buffering Relationships: is a type of calcium ion binding involved in regulation of cytosolic calcium ion concentration [GO:0099510]; is part of regulation of postsynaptic cytosolic calcium ion concentration [GO:0099566]; occurs in postsynaptic cytosol [GO:0099524] References: PMID:24442513, PMID:26190970 Definition: The directed change of free calcium ion concentration in the postsynaptic cytosol via the reversible binding of calcium ions to calcium-binding proteins in the cytosol thereby modulating the spatial and temporal dynamics of changes in postsynaptic cytosolic calcium concentrations.